cardioblast migration [GO:0003260] (biological process) Sources: GOC:mtg_heart Definition: The orderly movement of a cardiac progenitor cell to form the heart field. Cardiac progenitor cells are non-terminally differentiated, mesoderm-derived cells that are committed to differentiate into cells of the heart. A cardioblast is a cardiac precursor cell. It is a cell that has been committed to a cardiac fate, but will undergo more cell division rather than terminally differentiating. Relationships: is a type of cell migration involved in heart formation [GO:0060974] Subtypes: cardioblast anterior-lateral migration [GO:0003259], cardioblast migration to the midline involved in heart field formation [GO:0060975]